{
  "gene": "UniProtKB:Q2M2W7",
  "term_label": "Unknown cellular component",
  "gene_symbol": "C17orf58",
  "gene_name": "UPF0450 protein C17orf58",
  "term_id": "UNKNOWN:0003"
}